{
  "gene_symbol": "CFLAR",
  "gene": "UniProtKB:O15519",
  "gene_name": "CASP8 and FADD-like apoptosis regulator",
  "term_id": "GO:0006915",
  "term_label": "apoptotic process"
}